{
  "gene_name": "Translin",
  "term_id": "UNKNOWN:0002",
  "gene": "UniProtKB:Q15631",
  "term_label": "Unknown biological process",
  "gene_symbol": "TSN"
}